{
  "term_label": "keratin filament",
  "gene": "UniProtKB:Q9NSB4",
  "term_id": "GO:0045095",
  "gene_name": "Keratin, type II cuticular Hb2",
  "gene_symbol": "KRT82"
}